{
  "term_label": "olfactory receptor activity",
  "term_id": "GO:0004984",
  "gene_name": "Olfactory receptor 52E2",
  "gene_symbol": "OR52E2",
  "gene": "UniProtKB:Q8NGJ4"
}